K11-linked deubiquitinase activity [GO:0180017] (molecular function) References: PMID:26412298 Relationships: is_a deubiquitinase activity [GO:0101005] Definition: Hydrolysis of a ubiquitin unit from a ubiquitinated protein linked via the Lys11 residue of ubiquitin.